{
  "gene_name": "Stanniocalcin-1",
  "gene": "UniProtKB:P52823",
  "term_label": "Unknown molecular function",
  "gene_symbol": "STC1",
  "term_id": "UNKNOWN:0001"
}